{
  "gene": "UniProtKB:P11226",
  "gene_symbol": "MBL2",
  "term_label": "multivesicular body",
  "term_id": "GO:0005771",
  "gene_name": "Mannose-binding protein C"
}